{
  "gene_name": "Leucine-rich repeat serine_threonine-protein kinase 1",
  "term_id": "GO:0004674",
  "gene": "UniProtKB:Q38SD2",
  "gene_symbol": "LRRK1",
  "term_label": "protein serine/threonine kinase activity"
}